{
  "term_label": "actin filament binding",
  "term_id": "GO:0051015",
  "gene_name": "Unconventional myosin-Vc",
  "gene": "UniProtKB:Q9NQX4",
  "gene_symbol": "MYO5C"
}